{
  "term_label": "Unknown molecular function",
  "gene_symbol": "USP20",
  "gene": "UniProtKB:Q9Y2K6",
  "gene_name": "Ubiquitin carboxyl-terminal hydrolase 20",
  "term_id": "UNKNOWN:0001"
}